cyclic-GMP-AMP transmembrane transporter activity [GO:0140360] (molecular function) Definition: Enables the transfer of cyclic-GMP-AMP from one side of a membrane to the other. References: PMID:31126740 Relationships: is a type of adenine nucleotide transmembrane transporter activity [GO:0000295]; is a type of guanine nucleotide transmembrane transporter activity [GO:0001409]; is a type of purine ribonucleotide transmembrane transporter activity [GO:0005346]